diacylglycerol biosynthetic process [GO:0006651] (biological process) Regulation: regulated by regulation of diacylglycerol biosynthetic process [GO:1900480]; negatively regulated by negative regulation of diacylglycerol biosynthetic process [GO:1900481]; positively regulated by GO:1900482 Definition: The chemical reactions and pathways resulting in the formation of diacylglycerol, a glyceride in which any two of the R groups (positions not specified) are acyl groups while the remaining R group can be either H or an alkyl group. Sources: GOC:curators Relationships: is a type of diacylglycerol metabolic process [GO:0046339]; is a type of acylglycerol biosynthetic process [GO:0046463] Also known as: diacylglycerol anabolism, diacylglycerol biosynthesis, diacylglycerol formation, diacylglycerol synthesis, diglyceride biosynthesis